{
  "term_id": "GO:0005681",
  "term_label": "spliceosomal complex",
  "gene_symbol": "RBMY1D",
  "gene_name": "RNA-binding motif protein, Y chromosome, family 1 member D",
  "gene": "UniProtKB:P0C7P1"
}